{
  "term_label": "cytoplasm",
  "gene_symbol": "DOCK1",
  "gene_name": "Dedicator of cytokinesis protein 1",
  "gene": "UniProtKB:Q14185",
  "term_id": "GO:0005737"
}